{
  "gene": "UniProtKB:Q6BDI9",
  "gene_symbol": "REP15",
  "term_id": "UNKNOWN:0001",
  "term_label": "Unknown molecular function",
  "gene_name": "Rab15 effector protein"
}